response to reverse transcriptase inhibitor [GO:0061479] (biological process) Relationships: is a type of response to antibiotic [GO:0046677] Sources: GOC:dph Definition: Any process that results in a change in state or activity of a cell or an organism (in terms of movement, secretion, enzyme production, gene expression, etc.) as a result of a reverse transcriptase inhibitor stimulus.